{
  "term_label": "EMC complex",
  "gene_symbol": "MMGT1",
  "gene": "UniProtKB:Q8N4V1",
  "gene_name": "ER membrane protein complex subunit 5",
  "term_id": "GO:0072546"
}